{
  "term_id": "GO:0070488",
  "term_label": "neutrophil aggregation",
  "gene_name": "Protein S100-A9",
  "gene": "UniProtKB:P06702",
  "gene_symbol": "S100A9"
}